collagen type XIV trimer [GO:0005596] (cellular component) References: PMID:21421911 Relationships: is a type of FACIT collagen trimer [GO:0005593] Definition: A collagen homotrimer of alpha1(XIV) chains; type XIV collagen triple helices may link sheet-forming or fibrillar collagens to other structures.